{
  "term_id": "GO:0045296",
  "term_label": "cadherin binding",
  "gene_symbol": "CDH15",
  "gene": "UniProtKB:P55291",
  "gene_name": "Cadherin-15"
}